{
  "gene_name": "Laminin subunit gamma-3",
  "term_label": "extracellular matrix structural constituent",
  "gene": "UniProtKB:Q9Y6N6",
  "gene_symbol": "LAMC3",
  "term_id": "GO:0005201"
}